{
  "gene_name": "Ubiquitin carboxyl-terminal hydrolase 19",
  "gene": "UniProtKB:O94966",
  "term_label": "Unknown molecular function",
  "term_id": "UNKNOWN:0001",
  "gene_symbol": "USP19"
}